{
  "gene_name": "Putative zinc finger protein 286B",
  "gene_symbol": "ZNF286B",
  "term_id": "GO:0006357",
  "term_label": "regulation of transcription by RNA polymerase II",
  "gene": "UniProtKB:P0CG31"
}